{
  "gene_name": "Dynein regulatory complex subunit 3",
  "term_id": "GO:0005929",
  "term_label": "cilium",
  "gene_symbol": "DRC3",
  "gene": "UniProtKB:Q9H069"
}